{
  "term_label": "mediator complex",
  "gene": "UniProtKB:O95402",
  "term_id": "GO:0016592",
  "gene_symbol": "MED26",
  "gene_name": "Mediator of RNA polymerase II transcription subunit 26"
}